{
  "term_id": "UNKNOWN:0002",
  "gene_name": "C2 calcium-dependent domain-containing protein 4C",
  "gene_symbol": "C2CD4C",
  "term_label": "Unknown biological process",
  "gene": "UniProtKB:Q8TF44"
}